D-sorbitol dehydrogenase (acceptor) activity [GO:0047833] (molecular function) Relationships: is a type of GO:0016614 Also known as: D-sorbitol dehydrogenase activity, D-sorbitol:(acceptor) 1-oxidoreductase activity, D-sorbitol:acceptor 1-oxidoreductase activity Sources: RHEA:21320 Definition: Catalysis of the reaction: D-sorbitol + acceptor = L-sorbose + reduced acceptor.